{
  "gene_name": "Transmembrane protein 108",
  "gene": "UniProtKB:Q6UXF1",
  "term_label": "endosome membrane",
  "term_id": "GO:0010008",
  "gene_symbol": "TMEM108"
}